{
  "gene_name": "Iron-sulfur cluster assembly 2 homolog, mitochondrial",
  "gene_symbol": "ISCA2",
  "term_label": "protein maturation",
  "term_id": "GO:0051604",
  "gene": "UniProtKB:Q86U28"
}